Rad51B-Rad51C complex [GO:0033066] (cellular component) Relationships: is a type of DNA recombinase mediator complex [GO:0033061]; is a type of GO:0140513 Also known as: BC complex Definition: A DNA recombinase mediator complex that contains the Rad51 paralogs RAD51B and RAD51C, or orthologs thereof. References: PMID:16093548, PMID:17114795 Sources: GOC:mah